{
  "gene": "UniProtKB:Q86XM0",
  "term_id": "GO:0048240",
  "gene_symbol": "CATSPERD",
  "term_label": "sperm capacitation",
  "gene_name": "Cation channel sperm-associated auxiliary subunit delta"
}